positive regulation of development, heterochronic [GO:0045962] (biological process) Definition: Any process that modulates the consistent predetermined time point at which an integrated living unit or organism progresses from an initial condition to a later condition and increases the rate at which this time point is reached. Sources: GOC:go_curators Also known as: up regulation of development, heterochronic, up-regulation of development, heterochronic, upregulation of development, heterochronic, activation of development, heterochronic, stimulation of development, heterochronic Relationships: is a type of GO:0040034 Subtypes: positive regulation of nematode larval development, heterochronic [GO:0090445]